spot adherens junction [GO:0005914] (cellular component) Also known as: dense plaque, punctum adherens Definition: A small cell-cell adherens junction assembled during the cellularization stage of insect embyrogenesis; spot adherens junctions later fuse to form the zonula adherens. Relationships: is a type of GO:0005912 References: PMID:11700298